{
  "term_label": "neuron differentiation",
  "term_id": "GO:0030182",
  "gene_name": "Reticulon-4",
  "gene": "UniProtKB:Q9NQC3",
  "gene_symbol": "RTN4"
}